{
  "gene": "UniProtKB:P20396",
  "gene_name": "Pro-thyrotropin-releasing hormone",
  "gene_symbol": "TRH",
  "term_label": "secretory granule",
  "term_id": "GO:0030141"
}